{
  "term_label": "Unknown molecular function",
  "gene": "UniProtKB:Q9H0K4",
  "gene_name": "Radial spoke head protein 6 homolog A",
  "term_id": "UNKNOWN:0001",
  "gene_symbol": "RSPH6A"
}